{
  "gene_name": "Prominin-1",
  "term_id": "UNKNOWN:0001",
  "gene": "UniProtKB:O43490",
  "gene_symbol": "PROM1",
  "term_label": "Unknown molecular function"
}